{
  "term_label": "Unknown molecular function",
  "gene": "UniProtKB:Q9H0W5",
  "gene_symbol": "CCDC8",
  "gene_name": "Coiled-coil domain-containing protein 8",
  "term_id": "UNKNOWN:0001"
}